{
  "gene_symbol": "GALM",
  "gene_name": "Galactose mutarotase",
  "term_label": "Unknown cellular component",
  "term_id": "UNKNOWN:0003",
  "gene": "UniProtKB:Q96C23"
}